{
  "gene": "UniProtKB:A0A087WT02",
  "term_id": "GO:0002250",
  "gene_name": "T cell receptor alpha variable 9-2",
  "gene_symbol": "TRAV9-2",
  "term_label": "adaptive immune response"
}